{
  "term_id": "UNKNOWN:0001",
  "gene_symbol": "C4orf45",
  "term_label": "Unknown molecular function",
  "gene": "UniProtKB:Q96LM5",
  "gene_name": "Uncharacterized protein C4orf45"
}